{
  "gene_symbol": "FNDC3A",
  "term_label": "spermatid development",
  "term_id": "GO:0007286",
  "gene_name": "Fibronectin type-III domain-containing protein 3A",
  "gene": "UniProtKB:Q9Y2H6"
}